{
  "term_label": "Unknown cellular component",
  "gene_symbol": "KRTAP12-2",
  "gene_name": "Keratin-associated protein 12-2",
  "term_id": "UNKNOWN:0003",
  "gene": "UniProtKB:P59991"
}